{
  "gene": "UniProtKB:Q9NPF2",
  "term_label": "sulfotransferase activity",
  "gene_symbol": "CHST11",
  "gene_name": "Carbohydrate sulfotransferase 11",
  "term_id": "GO:0008146"
}